{
  "term_id": "GO:0000978",
  "gene_name": "Zinc finger and SCAN domain-containing protein 22",
  "gene": "UniProtKB:P10073",
  "term_label": "RNA polymerase II cis-regulatory region sequence-specific DNA binding",
  "gene_symbol": "ZSCAN22"
}